{
  "gene_name": "Putative beta-actin-like protein 3",
  "gene_symbol": "POTEKP",
  "gene": "UniProtKB:Q9BYX7",
  "term_label": "actin filament",
  "term_id": "GO:0005884"
}